vestibular reflex [GO:0060005] (biological process) Subtypes: angular vestibuloocular reflex [GO:0060006], linear vestibuloocular reflex [GO:0060007] Relationships: is a type of GO:0060004 Definition: A reflex process in which a response to an angular or linear acceleration stimulus begins with an afferent nerve impulse from a receptor in the inner ear and ends with the compensatory action of eye muscles. Signaling never reaches a level of consciousness. References: PMID:11784757